{
  "gene_symbol": "SNAPIN",
  "gene": "UniProtKB:O95295",
  "gene_name": "SNARE-associated protein Snapin",
  "term_id": "GO:0030141",
  "term_label": "secretory granule"
}